asexual sporulation resulting in formation of a cellular spore [GO:0043936] (biological process) Definition: The formation of a cellular spore derived from the products of mitosis. A cellular spore is a cell form that can be used for dissemination, for survival of adverse conditions because of its heat and desiccation resistance, and/or for reproduction. Sources: GOC:pamgo_curators Also known as: asexual sporulation resulting in the formation of a viable spore, asexual reproduction resulting in the formation of a cellular spore Relationships: is a type of sporulation resulting in formation of a cellular spore [GO:0030435]; is a type of asexual sporulation [GO:0030436] Subtypes: GO:0001410, sporangiospore formation [GO:0034300], endospore formation [GO:0034301], akinete formation [GO:0034302], myxospore formation [GO:0034303], actinomycete-type spore formation [GO:0034304], aeciospore formation [GO:0075247], uredospore formation [GO:0075251], teliospore formation [GO:0075255] Regulation: regulated by regulation of asexual sporulation resulting in formation of a cellular spore [GO:0043943]; negatively regulated by negative regulation of asexual sporulation resulting in formation of a cellular spore [GO:0043944]; positively regulated by positive regulation of asexual sporulation resulting in formation of a cellular spore [GO:0043945]